{
  "gene": "UniProtKB:Q6UWQ7",
  "term_label": "extracellular space",
  "gene_symbol": "IGFL2",
  "term_id": "GO:0005615",
  "gene_name": "Insulin growth factor-like family member 2"
}